{
  "gene_name": "Cytochrome P450 1B1",
  "gene_symbol": "CYP1B1",
  "gene": "UniProtKB:Q16678",
  "term_label": "oxidoreductase activity, acting on paired donors, with incorporation or reduction of molecular oxygen, reduced flavin or flavoprotein as one donor, and incorporation of one atom of oxygen",
  "term_id": "GO:0016712"
}